{
  "gene_name": "Retinoic acid receptor RXR-beta",
  "term_label": "cell differentiation",
  "gene_symbol": "RXRB",
  "gene": "UniProtKB:P28702",
  "term_id": "GO:0030154"
}